{
  "gene_symbol": "PTPRT",
  "term_id": "GO:0004725",
  "gene": "UniProtKB:O14522",
  "gene_name": "Receptor-type tyrosine-protein phosphatase T",
  "term_label": "protein tyrosine phosphatase activity"
}